{
  "gene_name": "Leucine-rich repeat-containing protein 74A",
  "term_label": "Unknown biological process",
  "gene": "UniProtKB:Q0VAA2",
  "term_id": "UNKNOWN:0002",
  "gene_symbol": "LRRC74A"
}